starch granule initiation [GO:0062052] (biological process) Relationships: is_a starch biosynthetic process [GO:0019252] References: PMID:28684429 Definition: The sequence of events that initiates (or primes) the synthesis of semi-crystalline starch granules within photosynthetic chloroplasts or non-photosynthetic amyloplasts.